{
  "gene": "UniProtKB:Q96T58",
  "gene_name": "Msx2-interacting protein",
  "term_id": "GO:0005634",
  "term_label": "nucleus",
  "gene_symbol": "SPEN"
}